{
  "gene_symbol": "H1-2",
  "term_id": "GO:0000791",
  "gene": "UniProtKB:P16403",
  "gene_name": "Histone H1.2",
  "term_label": "euchromatin"
}